{
  "gene": "UniProtKB:Q9Y2H9",
  "term_label": "intracellular signal transduction",
  "term_id": "GO:0035556",
  "gene_symbol": "MAST1",
  "gene_name": "Microtubule-associated serine_threonine-protein kinase 1"
}